18-methylnonadec-1-ene biosynthetic process [GO:1900881] (BP) Regulation: regulated by GO:1900950; negatively regulated by negative regulation of 18-methylnonadec-1-ene biosynthetic process [GO:1900951]; positively regulated by positive regulation of 18-methylnonadec-1-ene biosynthetic process [GO:1900952] Also known as: 18-methylnonadec-1-ene anabolism, 18-methylnonadec-1-ene biosynthesis, 18-methylnonadec-1-ene formation, 18-methylnonadec-1-ene synthesis Sources: GOC:TermGenie, GOC:mengo_curators Relationships: is a type of alkene biosynthetic process [GO:0043450]; is a type of 18-methylnonadec-1-ene metabolic process [GO:1900880] Definition: The chemical reactions and pathways resulting in the formation of 18-methylnonadec-1-ene.